{
  "term_id": "UNKNOWN:0003",
  "term_label": "Unknown cellular component",
  "gene_symbol": "RAB39B",
  "gene_name": "Ras-related protein Rab-39B",
  "gene": "UniProtKB:Q96DA2"
}